snRNA binding [GO:0017069] (MF) Definition: Binding to a small nuclear RNA (snRNA). Relationships: is a type of RNA binding [GO:0003723] Also known as: small nuclear RNA binding, base pairing with snRNA Subtypes: U6 snRNA binding [GO:0017070], GO:0030566, U1 snRNA binding [GO:0030619], GO:0030620, U4 snRNA binding [GO:0030621], U4atac snRNA binding [GO:0030622], U5 snRNA binding [GO:0030623], U6atac snRNA binding [GO:0030624], U11 snRNA binding [GO:0030625], U12 snRNA binding [GO:0030626], GO:0035614, GO:0071209, GO:0097322 Sources: GOC:mah